{
  "gene_symbol": "LLGL1",
  "gene_name": "Lethal(2) giant larvae protein homolog 1",
  "term_label": "GTPase activator activity",
  "gene": "UniProtKB:Q15334",
  "term_id": "GO:0005096"
}